{
  "term_label": "G protein-coupled receptor signaling pathway",
  "gene_symbol": "OR5AP2",
  "gene": "UniProtKB:Q8NGF4",
  "term_id": "GO:0007186",
  "gene_name": "Olfactory receptor 5AP2"
}